(+)-kotanin catabolic process [GO:1900595] (biological process) Sources: GOC:TermGenie, GOC:di Relationships: is a type of secondary metabolite catabolic process [GO:0090487] Definition: The chemical reactions and pathways resulting in the breakdown of (+)-kotanin. Also known as: (+)-kotanin breakdown, (+)-kotanin catabolism, (+)-kotanin degradation